{
  "gene": "UniProtKB:P49848",
  "gene_symbol": "TAF6",
  "gene_name": "Transcription initiation factor TFIID subunit 6",
  "term_label": "RNA polymerase II preinitiation complex assembly",
  "term_id": "GO:0051123"
}